{
  "term_label": "extracellular space",
  "gene": "UniProtKB:P21781",
  "gene_symbol": "FGF7",
  "gene_name": "Fibroblast growth factor 7",
  "term_id": "GO:0005615"
}